{
  "gene_name": "Transcriptional activator Myb",
  "term_label": "nucleus",
  "gene": "UniProtKB:P10242",
  "term_id": "GO:0005634",
  "gene_symbol": "MYB"
}